{
  "gene_symbol": "ANO8",
  "term_id": "UNKNOWN:0002",
  "term_label": "Unknown biological process",
  "gene": "UniProtKB:Q9HCE9",
  "gene_name": "Anoctamin-8"
}